{
  "term_label": "Unknown molecular function",
  "gene_symbol": "PEBP1",
  "gene": "UniProtKB:P30086",
  "gene_name": "Phosphatidylethanolamine-binding protein 1",
  "term_id": "UNKNOWN:0001"
}